{
  "gene": "UniProtKB:Q86VI3",
  "gene_name": "Ras GTPase-activating-like protein IQGAP3",
  "term_label": "GTPase activator activity",
  "gene_symbol": "IQGAP3",
  "term_id": "GO:0005096"
}